basement membrane/interstitial matrix interface [GO:0140086] (CC) Relationships: is a type of extracellular matrix [GO:0031012] Definition: The structure located at the interface of the basement membrane and interstitial extracellular matrix and anchoring the two types of ECM to one another. References: PMID:19945621, PMID:26377767, PMID:7767545, PMID:9334230